{
  "gene": "UniProtKB:Q8N7S2",
  "term_label": "Unknown molecular function",
  "term_id": "UNKNOWN:0001",
  "gene_symbol": "DNAJC5G",
  "gene_name": "DnaJ homolog subfamily C member 5G"
}